enzyme-thiol transhydrogenase (glutathione-disulfide) activity [GO:0047142] (molecular function) Sources: EC:1.8.4.7, MetaCyc:1.8.4.7-RXN Also known as: enzyme-thiol transhydrogenase (glutathione-disulphide) activity, enzyme-thiol transhydrogenase (oxidized-glutathione) activity, [xanthine-dehydrogenase]:oxidized-glutathione S-oxidoreductase activity, glutathione-dependent thiol:disulfide oxidoreductase activity, thiol:disulfide oxidoreductase activity, thiol:disulphide oxidoreductase activity, xanthine-dehydrogenase:glutathione-disulfide S-oxidoreductase activity, xanthine-dehydrogenase:oxidized-glutathione S-oxidoreductase activity Relationships: is a type of oxidoreductase activity, acting on a sulfur group of donors, disulfide as acceptor [GO:0016671] Definition: Catalysis of the reaction: oxidized glutathione + [xanthine dehydrogenase] = reduced glutathione + xanthine-oxidase.